{
  "gene_name": "Neurturin",
  "gene": "UniProtKB:Q99748",
  "term_id": "GO:0008083",
  "term_label": "growth factor activity",
  "gene_symbol": "NRTN"
}